RNA 5'-end processing [GO:0000966] (BP) Definition: Any process involved in forming the mature 5' end of an RNA molecule. Sources: GOC:krc Also known as: RNA 5' end processing Relationships: is a type of RNA processing [GO:0006396] Subtypes: GO:0000964, rRNA 5'-end processing [GO:0000967], RNA capping [GO:0036260], tRNA 5'-end processing [GO:0099116]